{
  "term_id": "GO:0007218",
  "term_label": "neuropeptide signaling pathway",
  "gene_name": "Somatostatin receptor type 4",
  "gene_symbol": "SSTR4",
  "gene": "UniProtKB:P31391"
}